{
  "gene_symbol": "SLC39A13",
  "gene_name": "Zinc transporter ZIP13",
  "term_label": "zinc ion transmembrane transport",
  "gene": "UniProtKB:Q96H72",
  "term_id": "GO:0071577"
}